{
  "term_label": "DNA-directed RNA polymerase activity",
  "gene_name": "DNA-directed RNA polymerase II subunit RPB3",
  "term_id": "GO:0003899",
  "gene": "UniProtKB:P19387",
  "gene_symbol": "POLR2C"
}